{
  "term_label": "DNA-binding transcription factor activity, RNA polymerase II-specific",
  "gene": "UniProtKB:Q9Y2H8",
  "term_id": "GO:0000981",
  "gene_name": "Zinc finger protein 510",
  "gene_symbol": "ZNF510"
}